{
  "gene_symbol": "KRBA1",
  "gene": "UniProtKB:A5PL33",
  "term_label": "Unknown molecular function",
  "term_id": "UNKNOWN:0001",
  "gene_name": "Protein KRBA1"
}